{
  "term_id": "GO:0006612",
  "gene_name": "Probable palmitoyltransferase ZDHHC11B",
  "gene_symbol": "ZDHHC11B",
  "term_label": "protein targeting to membrane",
  "gene": "UniProtKB:P0C7U3"
}